{
  "gene_symbol": "SLC25A2",
  "gene_name": "Mitochondrial ornithine transporter 2",
  "gene": "UniProtKB:Q9BXI2",
  "term_id": "GO:0000064",
  "term_label": "L-ornithine transmembrane transporter activity"
}